{
  "gene_symbol": "EPN2",
  "gene": "UniProtKB:O95208",
  "term_label": "endosome",
  "term_id": "GO:0005768",
  "gene_name": "Epsin-2"
}